negative regulation of pheromone response MAPK cascade [GO:0180040] (biological process) Sources: GOC:vw Definition: Any process that stops, prevents or reduces the frequency, rate or extent of a pheromone response MAPK cascade. Relationships: is a type of GO:0043409; is a type of regulation of pheromone response MAPK cascade [GO:0180039]; negatively regulates pheromone response MAPK cascade [GO:0071507]